ATP-dependent histone chaperone activity [GO:0140674] (molecular function) Relationships: is a type of GO:0140096; is a type of ATP-dependent chromatin remodeler activity [GO:0140658]; is a type of histone chaperone activity [GO:0140713] Subtypes: ATP-dependent H3-H4 histone complex chaperone activity [GO:0140665], ATP-dependent H2AZ histone chaperone activity [GO:0140849] Definition: Binding to and carrying a histone or a histone complex to unload or deposit it as a nucleosome, driven by ATP hydrolysis. Also known as: ATP-dependent histone loader activity, ATP-dependent histone unloader activity, histone loader activity, histone loading activity, histone unloader activity, histone unloading activity, nucleosome remodeling activity References: PMID:26459557